negative regulation of calcium ion-dependent exocytosis [GO:0045955] (biological process) Relationships: is a type of regulation of calcium ion-dependent exocytosis [GO:0017158]; is a type of negative regulation of regulated secretory pathway [GO:1903306]; negatively regulates GO:0017156 Also known as: down regulation of calcium ion-dependent exocytosis, down-regulation of calcium ion-dependent exocytosis, downregulation of calcium ion-dependent exocytosis, inhibition of calcium ion-dependent exocytosis Subtypes: negative regulation of calcium ion-dependent exocytosis of neurotransmitter [GO:1903234], negative regulation of dense core granule exocytosis [GO:1905414] Definition: Any process that stops, prevents, or reduces the frequency, rate or extent of calcium ion-dependent exocytosis. Sources: GOC:go_curators